{
  "gene_symbol": "GCSAM",
  "gene_name": "Germinal center-associated signaling and motility protein",
  "term_id": "UNKNOWN:0003",
  "term_label": "Unknown cellular component",
  "gene": "UniProtKB:Q8N6F7"
}